GPCR taste receptor activity [GO:0090681] (molecular function) Also known as: G-protein coupled taste receptor activity, G-protein-coupled taste receptor activity Sources: GOC:hat, GOC:tb Subtypes: umami taste receptor activity [GO:0033042], GPCR bitter taste receptor activity [GO:0090682], GPCR sweet taste receptor activity [GO:0090683] Definition: A G protein-coupled receptor activity that is responsible for the sense of taste. Relationships: is_a G protein-coupled receptor activity [GO:0004930]; is_a taste receptor activity [GO:0008527]